{
  "gene_name": "Zinc finger and BTB domain-containing protein 44",
  "gene": "UniProtKB:Q8NCP5",
  "term_label": "Unknown cellular component",
  "term_id": "UNKNOWN:0003",
  "gene_symbol": "ZBTB44"
}